specification of segmental identity, intercalary segment [GO:0035291] (biological process) Note: See also the fly_anatomy.ontology term 'intercalary segment ; FBbt:00000010'. Definition: The specification of the characteristic structures of the intercalary segment of the anterior head, following establishment of segment boundaries. Identity is considered to be the aggregate of characteristics by which a structure is recognized. Relationships: is a type of specification of segmental identity, head [GO:0007380]; is part of anterior head segmentation [GO:0035288] References: PMID:10477305 Sources: ISBN:0878932437